{
  "term_label": "calcium ion binding",
  "gene": "UniProtKB:P04054",
  "gene_name": "Phospholipase A2",
  "term_id": "GO:0005509",
  "gene_symbol": "PLA2G1B"
}